{
  "gene_symbol": "PDE10A",
  "term_id": "GO:0047555",
  "gene": "UniProtKB:Q9Y233",
  "gene_name": "cAMP and cAMP-inhibited cGMP 3',5'-cyclic phosphodiesterase 10A",
  "term_label": "3',5'-cyclic-GMP phosphodiesterase activity"
}